{
  "gene_name": "Coiled-coil domain-containing protein 25",
  "term_label": "Unknown cellular component",
  "gene": "UniProtKB:Q86WR0",
  "gene_symbol": "CCDC25",
  "term_id": "UNKNOWN:0003"
}